{
  "gene_symbol": "OSGIN2",
  "gene": "UniProtKB:Q9Y236",
  "gene_name": "Oxidative stress-induced growth inhibitor 2",
  "term_id": "GO:0030308",
  "term_label": "negative regulation of cell growth"
}